{
  "gene_name": "Histone H2A type 2-C",
  "term_id": "GO:0030527",
  "gene_symbol": "H2AC20",
  "gene": "UniProtKB:Q16777",
  "term_label": "structural constituent of chromatin"
}